{
  "term_id": "GO:0005096",
  "term_label": "GTPase activator activity",
  "gene_symbol": "SRGAP2",
  "gene_name": "SLIT-ROBO Rho GTPase-activating protein 2",
  "gene": "UniProtKB:O75044"
}